(RS)-norcoclaurine 6-O-methyltransferase activity [GO:0030786] (MF) Relationships: is a type of S-adenosylmethionine-dependent methyltransferase activity [GO:0008757] Also known as: S-adenosyl-L-methionine:(RS)-norcoclaurine 6-O-methyltransferase activity Sources: EC:2.1.1.128 Definition: Catalysis of the reaction: S-adenosyl-L-methionine + (RS)-norcoclaurine = S-adenosyl-L-homocysteine + (RS)-coclaurine.